{
  "gene": "UniProtKB:Q674R7",
  "term_label": "phagophore assembly site",
  "gene_name": "Autophagy-related protein 9B",
  "gene_symbol": "ATG9B",
  "term_id": "GO:0000407"
}